{
  "term_label": "monoatomic ion transmembrane transport",
  "term_id": "GO:0034220",
  "gene_name": "Neuronal acetylcholine receptor subunit beta-3",
  "gene": "UniProtKB:Q05901",
  "gene_symbol": "CHRNB3"
}